{
  "term_label": "Unknown biological process",
  "gene_name": "Protein FAM162B",
  "gene_symbol": "FAM162B",
  "gene": "UniProtKB:Q5T6X4",
  "term_id": "UNKNOWN:0002"
}